{
  "gene_symbol": "SHISA7",
  "gene": "UniProtKB:A6NL88",
  "gene_name": "Protein shisa-7",
  "term_label": "dendritic spine membrane",
  "term_id": "GO:0032591"
}